{
  "gene_name": "Ankyrin repeat and MYND domain-containing protein 1",
  "gene": "UniProtKB:Q9P2S6",
  "term_id": "UNKNOWN:0002",
  "term_label": "Unknown biological process",
  "gene_symbol": "ANKMY1"
}